mRNA N6-methyladenosine dioxygenase activity [GO:1990931] (molecular function) Definition: Catalysis of the oxidative demethylation of N6-methyladenosine RNA, with concomitant decarboxylation of 2-oxoglutarate and releases oxidized methyl group on N6-methyladenosine as formaldehyde. References: PMID:22002720, PMID:26458103 Relationships: is a type of oxidative RNA demethylase activity [GO:0035515] Also known as: mRNA N(6)-methyladenine demethylase, mRNA N(6)-methyladenosine dioxygenase activity, RNA N6-methyladenosine dioxygenase activity